complement receptor mediated signaling pathway [GO:0002430] (biological process) Relationships: is a type of immune response-activating cell surface receptor signaling pathway [GO:0002429] Sources: GOC:add, GO_REF:0000022, ISBN:0781735149 Subtypes: complement component C5a signaling pathway [GO:0038178] Definition: The series of molecular signals generated as a consequence of a component of the complement pathway binding to a complement receptor. Such components include both whole complement proteins and fragments of complement proteins generated through the activity of the complement pathway. Also known as: immune response-regulating cell surface receptor signalling pathway, complement receptor mediated signalling pathway